{
  "gene_name": "Fibroblast growth factor 12",
  "gene": "UniProtKB:P61328",
  "term_label": "nucleus",
  "term_id": "GO:0005634",
  "gene_symbol": "FGF12"
}